{
  "gene_symbol": "KIRREL3",
  "gene": "UniProtKB:Q8IZU9",
  "term_label": "cell adhesion molecule binding",
  "term_id": "GO:0050839",
  "gene_name": "Kin of IRRE-like protein 3"
}